{
  "gene_symbol": "IGF2BP2",
  "term_id": "GO:0010494",
  "gene_name": "Insulin-like growth factor 2 mRNA-binding protein 2",
  "term_label": "cytoplasmic stress granule",
  "gene": "UniProtKB:Q9Y6M1"
}